{
  "term_id": "GO:0045727",
  "gene_name": "Protein Largen",
  "gene_symbol": "PRR16",
  "term_label": "positive regulation of translation",
  "gene": "UniProtKB:Q569H4"
}